{
  "term_label": "U4 snRNP",
  "gene": "UniProtKB:P62308",
  "gene_symbol": "SNRPG",
  "gene_name": "Small nuclear ribonucleoprotein G",
  "term_id": "GO:0005687"
}